{
  "gene": "UniProtKB:Q6ZVE7",
  "gene_name": "Vesicle transport protein GOT1A",
  "gene_symbol": "GOLT1A",
  "term_label": "Unknown molecular function",
  "term_id": "UNKNOWN:0001"
}